{
  "gene_name": "Nipped-B-like protein",
  "term_id": "GO:0003682",
  "gene_symbol": "NIPBL",
  "gene": "UniProtKB:Q6KC79",
  "term_label": "chromatin binding"
}